meiotic telophase II [GO:0007139] (biological process) Definition: The cell cycle phase which follows anaphase II of meiosis and during which the chromosomes arrive at the poles of the cell and the division of the cytoplasm starts. Note: Note that this term should not be used for direct annotation. If you are trying to make an annotation to x phase, it is likely that the correct annotation is 'regulation of x/y phase transition' or to a process which occurs during the reported phase (i.e mitotic DNA replication for mitotic S-phase). To capture the phase when a specific location or process is observed, the phase term can be used in an annotation extension (PMID:24885854) applied to a cellular component term (with the relation exists_during) or a biological process term (with the relation happens_during). Relationships: is a type of telophase [GO:0051326]; is a type of meiosis II cell cycle phase [GO:0098765] Sources: GOC:mtg_cell_cycle